{
  "gene_symbol": "AHRR",
  "term_label": "aryl hydrocarbon receptor complex",
  "term_id": "GO:0034751",
  "gene": "UniProtKB:A9YTQ3",
  "gene_name": "Aryl hydrocarbon receptor repressor"
}